{
  "term_label": "Unknown molecular function",
  "gene": "UniProtKB:Q86W25",
  "gene_name": "NACHT, LRR and PYD domains-containing protein 13",
  "gene_symbol": "NLRP13",
  "term_id": "UNKNOWN:0001"
}